{
  "term_id": "GO:0006805",
  "gene_symbol": "CYP2F1",
  "term_label": "xenobiotic metabolic process",
  "gene_name": "Cytochrome P450 2F1",
  "gene": "UniProtKB:P24903"
}